{
  "term_label": "amyloid-beta binding",
  "gene_name": "Amyloid-beta A4 precursor protein-binding family A member 2",
  "gene_symbol": "APBA2",
  "term_id": "GO:0001540",
  "gene": "UniProtKB:Q99767"
}